{
  "gene_symbol": "EME1",
  "gene": "UniProtKB:Q96AY2",
  "term_label": "double-strand break repair",
  "gene_name": "Crossover junction endonuclease EME1",
  "term_id": "GO:0006302"
}